zygote asymmetric cell division [GO:0010070] (biological process) Also known as: zygote asymmetric cytokinesis Subtypes: zygote asymmetric cytokinesis in embryo sac [GO:0010069] Sources: GOC:tb Definition: The division of the zygote into two daughter cells that will adopt developmentally distinct potentials. Relationships: is a type of GO:0008356